{
  "gene_symbol": "CYP2A13",
  "term_id": "GO:0020037",
  "term_label": "heme binding",
  "gene_name": "Cytochrome P450 2A13",
  "gene": "UniProtKB:Q16696"
}